{
  "term_id": "GO:0045087",
  "gene": "UniProtKB:Q30KQ6",
  "gene_name": "Beta-defensin 114",
  "gene_symbol": "DEFB114",
  "term_label": "innate immune response"
}